regulation of calcium ion import into sarcoplasmic reticulum [GO:1902080] (biological process) Subtypes: negative regulation of calcium ion import into sarcoplasmic reticulum [GO:1902081], positive regulation of calcium ion import into sarcoplasmic reticulum [GO:1902082] Relationships: is a type of regulation of intracellular transport [GO:0032386]; is a type of regulation of calcium ion transport [GO:0051924]; regulates calcium ion import into sarcoplasmic reticulum [GO:1990036] Definition: Any process that modulates the frequency, rate or extent of calcium ion import into sarcoplasmic reticulum. References: PMID:8349590 Sources: GOC:BHF, GOC:TermGenie, GOC:rl